muscle atrophy [GO:0014889] (biological process) Relationships: is_a muscle adaptation [GO:0043500] Definition: A process, occurring in the muscle, that is characterized by a decrease in protein content, fiber diameter, force production and fatigue resistance in response to different conditions such as starvation, aging and disuse. Note: GO:0014889 should only be used for annotation when muscle atrophy is a normal physiological process and not a disease process. Regulation: regulated by regulation of muscle atrophy [GO:0014735]; RO_0002212 by negative regulation of muscle atrophy [GO:0014736]; positively regulated by positive regulation of muscle atrophy [GO:0014737] Subtypes: GO:0014890, striated muscle atrophy [GO:0014891] Sources: GOC:mtg_muscle